cell-cell signaling involved in mammary gland development [GO:0060764] (biological process) Definition: Any process that mediates the transfer of information from one cell to another and contributes to the progression of the mammary gland, from its initial state to the mature structure. Sources: GOC:dph Also known as: cell-cell signalling involved in mammary gland development Relationships: is a type of cell-cell signaling [GO:0007267]; is part of mammary gland development [GO:0030879]